{
  "term_label": "phosphatidylinositol-mediated signaling",
  "term_id": "GO:0048015",
  "gene_name": "1-phosphatidylinositol 4,5-bisphosphate phosphodiesterase gamma-1",
  "gene_symbol": "PLCG1",
  "gene": "UniProtKB:P19174"
}